{
  "gene_name": "BAG family molecular chaperone regulator 4",
  "term_id": "GO:0051087",
  "term_label": "protein-folding chaperone binding",
  "gene": "UniProtKB:O95429",
  "gene_symbol": "BAG4"
}